preribosome, large subunit precursor [GO:0030687] (cellular component) Definition: A preribosomal complex consisting of 27SA, 27SB, and/or 7S pre-rRNA, 5S rRNA, ribosomal proteins including late-associating large subunit proteins, and associated proteins; a precursor of the eukaryotic cytoplasmic large ribosomal subunit. References: PMID:10567516 Note: Note that this complex is 66S in Saccharomyces. Also known as: 66S preribosome Relationships: is_a GO:0030684